tetrapyrrole biosynthetic process from glutamate [GO:0033526] (biological process) Also known as: tetrapyrrole anabolism from glutamate, tetrapyrrole biosynthesis from glutamate, tetrapyrrole formation from glutamate, tetrapyrrole synthesis from glutamate Regulation: regulated by regulation of tetrapyrrole biosynthetic process from glutamate [GO:1901410]; negatively regulated by negative regulation of tetrapyrrole biosynthetic process from glutamate [GO:1901411]; positively regulated by positive regulation of tetrapyrrole biosynthetic process from glutamate [GO:1901412] Sources: GOC:mah, MetaCyc:PWY-5188 Relationships: is a type of glutamate metabolic process [GO:0006536]; is a type of tetrapyrrole biosynthetic process [GO:0033014] Definition: The chemical reactions and pathways leading to the formation of tetrapyrroles, natural pigments containing four pyrrole rings joined by one-carbon units linking position 2 of one pyrrole ring to position 5 of the next, from other compounds, including L-glutamate. Subtypes: protoporphyrinogen IX biosynthetic process from glutamate [GO:0019353]